{
  "term_label": "RNA polymerase II cis-regulatory region sequence-specific DNA binding",
  "gene": "UniProtKB:Q8WYA1",
  "gene_name": "Basic helix-loop-helix ARNT-like protein 2",
  "gene_symbol": "BMAL2",
  "term_id": "GO:0000978"
}